{
  "term_id": "GO:0005483",
  "term_label": "soluble NSF attachment protein activity",
  "gene": "UniProtKB:P54920",
  "gene_name": "Alpha-soluble NSF attachment protein",
  "gene_symbol": "NAPA"
}